chemorepulsion of branchiomotor axon [GO:0021793] (biological process) References: PMID:14699587 Sources: GOC:cls, GOC:dgh, GOC:dph, GOC:jid, GO_REF:0000021 Definition: The process in which a branchiomotor neuron growth cone is directed to a specific target site in response to a repulsive chemical cue. Branchiomotor neurons are located in the hindbrain and innervate branchial arch-derived muscles that control jaw movements, facial expression, the larynx, and the pharynx. Subtypes: GO:0021787, chemorepulsion of branchiomotor neuron axon in branchial arch mesenchyme [GO:0021790] Relationships: is a type of chemorepulsion of axon [GO:0061643]; BFO_0000050 branchiomotor neuron axon guidance [GO:0021785] Also known as: negative chemotaxis of branchiomotor axon